{
  "gene_name": "Cancer-related nucleoside-triphosphatase",
  "term_id": "UNKNOWN:0001",
  "gene_symbol": "NTPCR",
  "gene": "UniProtKB:Q9BSD7",
  "term_label": "Unknown molecular function"
}